negative regulation of protein-containing complex disassembly [GO:0043242] (biological process) Subtypes: negative regulation of SNARE complex disassembly [GO:0035541], negative regulation of translational termination [GO:0045904], negative regulation of termination of DNA-templated transcription [GO:0060567], negative regulation of DNA recombinase disassembly [GO:0062110], negative regulation of autophagosome maturation [GO:1901097], negative regulation of protein depolymerization [GO:1901880] Sources: GOC:jl Also known as: down regulation of protein complex disassembly, down-regulation of protein complex disassembly, downregulation of protein complex disassembly, inhibition of protein complex disassembly, negative regulation of protein complex disassembly Relationships: is a type of regulation of protein-containing complex disassembly [GO:0043244]; is a type of negative regulation of cellular component organization [GO:0051129]; negatively regulates GO:0032984 Definition: Any process that stops, prevents, or reduces the frequency, rate or extent of protein complex disassembly, the disaggregation of a protein complex into its constituent components.